{
  "gene": "UniProtKB:Q9BXU9",
  "term_label": "Unknown molecular function",
  "gene_name": "Calcium-binding protein 8",
  "gene_symbol": "CALN1",
  "term_id": "UNKNOWN:0001"
}